{
  "term_label": "DNA-binding transcription factor activity, RNA polymerase II-specific",
  "gene": "UniProtKB:Q3KNW1",
  "term_id": "GO:0000981",
  "gene_symbol": "SNAI3",
  "gene_name": "Zinc finger protein SNAI3"
}